{
  "gene": "UniProtKB:Q8TEC5",
  "term_id": "GO:0008157",
  "term_label": "protein phosphatase 1 binding",
  "gene_symbol": "SH3RF2",
  "gene_name": "E3 ubiquitin-protein ligase SH3RF2"
}